{
  "gene_name": "Mothers against decapentaplegic homolog 4",
  "gene_symbol": "SMAD4",
  "gene": "UniProtKB:Q13485",
  "term_label": "regulation of transcription by RNA polymerase II",
  "term_id": "GO:0006357"
}